{
  "term_id": "GO:0050729",
  "term_label": "positive regulation of inflammatory response",
  "gene": "UniProtKB:Q08722",
  "gene_name": "Leukocyte surface antigen CD47",
  "gene_symbol": "CD47"
}